{
  "gene_symbol": "ZGLP1",
  "gene_name": "GATA-type zinc finger protein 1",
  "term_label": "Unknown molecular function",
  "term_id": "UNKNOWN:0001",
  "gene": "UniProtKB:P0C6A0"
}